{
  "term_id": "GO:0019005",
  "term_label": "SCF ubiquitin ligase complex",
  "gene": "UniProtKB:Q9UKT7",
  "gene_name": "F-box_LRR-repeat protein 3",
  "gene_symbol": "FBXL3"
}